mesenchymal stem cell differentiation involved in mesonephric nephron morphogenesis [GO:0061239] (biological process) Definition: The process in which a relatively unspecialized cell acquires specialized features of a mesenchymal stem cell that contributes to the shaping of a nephronin the mesonephros. A mesenchymal stem cell is a cell that retains the ability to divide and proliferate throughout life to provide progenitor cells that can differentiate into specialized mesenchymal cells. Sources: GOC:mtg_kidney_jan10 Relationships: is a type of GO:0061208; is a type of mesenchymal stem cell differentiation involved in nephron morphogenesis [GO:0072037]; is part of GO:0061228